{
  "gene": "UniProtKB:Q9H7N4",
  "gene_symbol": "SCAF1",
  "gene_name": "Splicing factor, arginine_serine-rich 19",
  "term_id": "GO:0099122",
  "term_label": "RNA polymerase II C-terminal domain binding"
}